{
  "gene_symbol": "RNF157",
  "term_id": "UNKNOWN:0002",
  "term_label": "Unknown biological process",
  "gene_name": "E3 ubiquitin ligase RNF157",
  "gene": "UniProtKB:Q96PX1"
}